enzyme inhibitor activity [GO:0004857] (molecular function) Subtypes: GO:0004858, GTPase inhibitor activity [GO:0005095], ornithine decarboxylase inhibitor activity [GO:0008073], DNA topoisomerase type II (double strand cut, ATP-hydrolyzing) inhibitor activity [GO:0008657], telomerase inhibitor activity [GO:0010521], cyclase inhibitor activity [GO:0010852], alpha-amylase inhibitor activity [GO:0015066], GO:0019210, phosphatase inhibitor activity [GO:0019212], GO:0030414, peroxidase inhibitor activity [GO:0036479], GO:0036487, histone deacetylase inhibitor activity [GO:0046811], GO:0046910, lipase inhibitor activity [GO:0055102], GO:0055104, GO:0055105, GO:0060241, polygalacturonase inhibitor activity [GO:0090353], ornithine carbamoyltransferase inhibitor activity [GO:0090369], GO:0140594, DNA strand exchange inhibitor activity [GO:0140620], GO:0140631, nuclease inhibitor activity [GO:0140721], RNA polymerase inhibitor activity [GO:0140870], L-lactate dehydrogenase inhibitor activity [GO:0160193], histone methyltransferase inhibitor activity [GO:0180000], RNA helicase inhibitor activity [GO:1990119], GO:1990624, ribonucleoside-diphosphate reductase inhibitor activity [GO:1990846] Also known as: metalloenzyme inhibitor activity Relationships: is a type of enzyme regulator activity [GO:0030234]; is a type of molecular function inhibitor activity [GO:0140678]; negatively regulates catalytic activity [GO:0003824] Sources: GOC:ai, GOC:ebc Definition: A molecular function regulator that reduces a catalytic activity. Note: This term should only be used in cases when the regulator directly interacts with the enzyme, but does not result in a covalent modification.